{
  "gene": "UniProtKB:P54756",
  "term_id": "GO:0030425",
  "gene_name": "Ephrin type-A receptor 5",
  "gene_symbol": "EPHA5",
  "term_label": "dendrite"
}